bacterial nucleoid DNA packaging [GO:0036386] (biological process) References: PMID:17097674, PMID:17360520 Sources: GOC:bf, GOC:bhm Also known as: chromosomal compaction, nucleoid compaction, prokaryotic DNA condensation Relationships: is a type of chromosome organization [GO:0051276]; occurs in bacterial nucleoid [GO:0043590] Definition: A process in which chromosomal DNA and associated proteins organize into a compact, orderly bacterial nucleoid. Often resulting in DNA supercoiling.